hepatocyte proliferation [GO:0072574] (biological process) Relationships: is a type of GO:0072575 Regulation: regulated by GO:2000345; negatively regulated by negative regulation of hepatocyte proliferation [GO:2000346]; positively regulated by positive regulation of hepatocyte proliferation [GO:2000347] Sources: CL:0000182, GOC:BHF, GOC:mah Definition: The multiplication or reproduction of hepatocytes, resulting in the expansion of a cell population. Hepatocytes form the main structural component of the liver. They are specialized epithelial cells that are organized into interconnected plates called lobules.